{
  "gene": "UniProtKB:Q92521",
  "gene_symbol": "PIGB",
  "gene_name": "GPI mannosyltransferase 3",
  "term_id": "GO:0005789",
  "term_label": "endoplasmic reticulum membrane"
}